ACP-dependent peptidyl-lysine N6-myristoyltransferase activity [GO:0140769] (molecular function) Definition: Catalysis of the reaction: L-lysyl-[protein] + tetradecanoyl-[ACP] = H+ + holo-[ACP] + N(6)-tetradecanoyl-L-lysyl-[protein]. References: PMID:32461253 Sources: RHEA:70611 Relationships: is a type of peptidyl-lysine N6-myristoyltransferase activity [GO:0018030]